{
  "gene_symbol": "KCTD16",
  "gene_name": "BTB_POZ domain-containing protein KCTD16",
  "gene": "UniProtKB:Q68DU8",
  "term_label": "regulation of G protein-coupled receptor signaling pathway",
  "term_id": "GO:0008277"
}